{
  "term_label": "nuclear pore",
  "gene": "UniProtKB:Q9H2T7",
  "gene_name": "Ran-binding protein 17",
  "gene_symbol": "RANBP17",
  "term_id": "GO:0005643"
}